{
  "gene": "UniProtKB:Q07001",
  "term_label": "monoatomic ion transmembrane transport",
  "term_id": "GO:0034220",
  "gene_symbol": "CHRND",
  "gene_name": "Acetylcholine receptor subunit delta"
}